{
  "gene_name": "Insulin",
  "gene_symbol": "INS",
  "term_label": "extracellular space",
  "gene": "UniProtKB:P01308",
  "term_id": "GO:0005615"
}